{
  "term_id": "GO:0005829",
  "gene_name": "Actin filament-associated protein 1-like 2",
  "term_label": "cytosol",
  "gene": "UniProtKB:Q8N4X5",
  "gene_symbol": "AFAP1L2"
}